{
  "term_label": "mitochondrial matrix",
  "gene_symbol": "FASTKD5",
  "gene_name": "FAST kinase domain-containing protein 5, mitochondrial",
  "gene": "UniProtKB:Q7L8L6",
  "term_id": "GO:0005759"
}